{
  "term_id": "UNKNOWN:0003",
  "gene_symbol": "A4GALT",
  "gene": "UniProtKB:Q9NPC4",
  "gene_name": "Lactosylceramide 4-alpha-galactosyltransferase",
  "term_label": "Unknown cellular component"
}